{
  "gene_symbol": "SIT1",
  "gene_name": "Signaling threshold-regulating transmembrane adapter 1",
  "gene": "UniProtKB:Q9Y3P8",
  "term_label": "kinase binding",
  "term_id": "GO:0019900"
}